{
  "gene": "UniProtKB:Q693B1",
  "gene_symbol": "KCTD11",
  "term_id": "UNKNOWN:0003",
  "gene_name": "BTB_POZ domain-containing protein KCTD11",
  "term_label": "Unknown cellular component"
}